{
  "gene": "UniProtKB:Q4V328",
  "term_label": "regulation of neurotransmitter receptor transport, endosome to postsynaptic membrane",
  "gene_symbol": "GRIPAP1",
  "term_id": "GO:0099152",
  "gene_name": "GRIP1-associated protein 1"
}